{
  "term_label": "intracellular protein transport",
  "term_id": "GO:0006886",
  "gene": "UniProtKB:Q9Y3B3",
  "gene_name": "Transmembrane emp24 domain-containing protein 7",
  "gene_symbol": "TMED7"
}